negative regulation of immature T cell proliferation [GO:0033087] (biological process) Subtypes: negative regulation of immature T cell proliferation in thymus [GO:0033088] Definition: Any process that stops, prevents, or reduces the frequency, rate or extent of immature T cell proliferation. Relationships: is_a regulation of immature T cell proliferation [GO:0033083]; is a type of negative regulation of T cell proliferation [GO:0042130]; negatively regulates immature T cell proliferation [GO:0033079] Sources: GOC:add, GOC:mah